{
  "gene_name": "Endophilin-A3",
  "term_id": "GO:0005829",
  "term_label": "cytosol",
  "gene": "UniProtKB:Q99963",
  "gene_symbol": "SH3GL3"
}